{
  "gene_name": "Alanine aminotransferase 1",
  "gene_symbol": "GPT",
  "gene": "UniProtKB:P24298",
  "term_id": "UNKNOWN:0002",
  "term_label": "Unknown biological process"
}